{
  "gene_name": "Protein S100-B",
  "term_id": "GO:0005634",
  "gene_symbol": "S100B",
  "term_label": "nucleus",
  "gene": "UniProtKB:P04271"
}